Harderian gland development [GO:0070384] (biological process) Note: Note that the Harderian gland is found in all terrestrial vertebrate groups, including amphibia, reptiles, birds, and mammals. However, it appears to be absent in certain mammals such as bats, cows, horses, and higher primates. Though largely absent in the adult human, it is present in the fetal and neonatal stages. Definition: The process whose specific outcome is the progression of the Harderian gland over time, from its formation to the mature structure. The Harderian gland is an anterior orbital structure usually associated with the nictitating membrane, and produces and secretes a variety of substances to the eye, depending upon the species. References: PMID:16856596, PMID:7559104 Sources: GOC:hjd Relationships: is a type of gland development [GO:0048732]